{
  "gene": "UniProtKB:Q96LL4",
  "term_label": "Unknown biological process",
  "gene_name": "Uncharacterized protein C8orf48",
  "gene_symbol": "C8orf48",
  "term_id": "UNKNOWN:0002"
}